{
  "gene": "UniProtKB:Q13526",
  "gene_symbol": "PIN1",
  "term_id": "UNKNOWN:0002",
  "gene_name": "Peptidyl-prolyl cis-trans isomerase NIMA-interacting 1",
  "term_label": "Unknown biological process"
}